{
  "gene_symbol": "KRTAP21-1",
  "term_label": "Unknown biological process",
  "term_id": "UNKNOWN:0002",
  "gene_name": "Keratin-associated protein 21-1",
  "gene": "UniProtKB:Q3LI58"
}